symbiont-mediated suppression of host cGAS-STING signal transduction [GO:0141074] (biological process) Definition: A process in which a virus interferes with, inhibits or disrupt a cGAS/STING signal transduction in the host organism. The host is defined as the larger of the organisms involved in a symbiotic interaction. References: PMID:26405230, PMID:27234299, PMID:29018427 Also known as: disruption of host cGAS-STING signal transduction, disruption of host cGAS-STING signaling, suppression of host cGAS-STING Relationships: is a type of symbiont-mediated suppression of cytoplasmic pattern recognition receptor signaling pathway [GO:0039537]